{
  "gene_symbol": "KIF12",
  "gene": "UniProtKB:Q96FN5",
  "term_id": "GO:0016887",
  "term_label": "ATP hydrolysis activity",
  "gene_name": "Kinesin-like protein KIF12"
}